{
  "gene_symbol": "ARMC9",
  "term_label": "cilium assembly",
  "gene": "UniProtKB:Q7Z3E5",
  "gene_name": "LisH domain-containing protein ARMC9",
  "term_id": "GO:0060271"
}